negative regulation of mitotic nuclear division [GO:0045839] (biological process) Also known as: down regulation of mitosis, down-regulation of mitosis, downregulation of mitosis, negative regulation of mitosis, inhibition of mitosis Sources: GOC:dph, GOC:go_curators, GOC:tb Subtypes: negative regulation of mitotic metaphase/anaphase transition [GO:0045841] Definition: Any process that stops, prevents or reduces the rate or extent of mitosis. Mitosis is the division of the eukaryotic cell nucleus to produce two daughter nuclei that, usually, contain the identical chromosome complement to their mother. Relationships: is a type of regulation of mitotic nuclear division [GO:0007088]; is a type of negative regulation of cell cycle process [GO:0010948]; is a type of GO:0045930; is a type of negative regulation of nuclear division [GO:0051784]; negatively regulates mitotic nuclear division [GO:0140014]